{
  "gene_name": "Zinc finger protein 284",
  "term_label": "Unknown cellular component",
  "term_id": "UNKNOWN:0003",
  "gene_symbol": "ZNF284",
  "gene": "UniProtKB:Q2VY69"
}